{
  "gene_name": "Small nuclear ribonucleoprotein Sm D1",
  "gene_symbol": "SNRPD1",
  "term_id": "GO:0034715",
  "term_label": "pICln-Sm protein complex",
  "gene": "UniProtKB:P62314"
}